{
  "term_label": "mRNA export from nucleus",
  "term_id": "GO:0006406",
  "gene_symbol": "ALYREF",
  "gene_name": "THO complex subunit 4",
  "gene": "UniProtKB:Q86V81"
}